{
  "term_label": "cell migration",
  "term_id": "GO:0016477",
  "gene_symbol": "CDH13",
  "gene_name": "Cadherin-13",
  "gene": "UniProtKB:P55290"
}